{
  "gene_name": "Microtubule-associated serine_threonine-protein kinase 4",
  "gene_symbol": "MAST4",
  "term_label": "intracellular signal transduction",
  "gene": "UniProtKB:O15021",
  "term_id": "GO:0035556"
}